{
  "term_id": "GO:0050431",
  "gene_name": "Transforming growth factor-beta receptor type 3-like protein",
  "gene": "UniProtKB:H3BV60",
  "term_label": "transforming growth factor beta binding",
  "gene_symbol": "TGFBR3L"
}